{
  "term_id": "GO:0000978",
  "gene_symbol": "HES4",
  "gene": "UniProtKB:Q9HCC6",
  "term_label": "RNA polymerase II cis-regulatory region sequence-specific DNA binding",
  "gene_name": "Transcription factor HES-4"
}